{
  "term_id": "UNKNOWN:0002",
  "gene_symbol": "TNFRSF8",
  "term_label": "Unknown biological process",
  "gene": "UniProtKB:P28908",
  "gene_name": "Tumor necrosis factor receptor superfamily member 8"
}